{
  "gene_name": "Spermatogenesis-associated protein 31A7",
  "gene": "UniProtKB:Q8IWB4",
  "term_id": "UNKNOWN:0002",
  "gene_symbol": "SPATA31A7",
  "term_label": "Unknown biological process"
}